antigenic variation [GO:0020033] (biological process) Also known as: surface antigen variation Definition: A process by which a symbiont evades the host adaptive immune response by changing antigenic determinants on the symbiont surface that are exposed to host antibodies. Relationships: is a type of symbiont-mediated evasion of host immune response [GO:0042783] References: PMID:29116635, PMID:37524976